{
  "term_label": "plasma membrane",
  "term_id": "GO:0005886",
  "gene": "UniProtKB:Q86VW2",
  "gene_name": "Rho guanine nucleotide exchange factor 25",
  "gene_symbol": "ARHGEF25"
}